{
  "gene_name": "THUMP domain-containing protein 2",
  "gene_symbol": "THUMPD2",
  "term_label": "tRNA methylation",
  "gene": "UniProtKB:Q9BTF0",
  "term_id": "GO:0030488"
}